{
  "term_id": "GO:0005085",
  "gene_symbol": "ARHGEF1",
  "term_label": "guanyl-nucleotide exchange factor activity",
  "gene": "UniProtKB:Q92888",
  "gene_name": "Rho guanine nucleotide exchange factor 1"
}